{
  "term_label": "tetrahydrofolate interconversion",
  "gene_name": "Bifunctional methylenetetrahydrofolate dehydrogenase_cyclohydrolase, mitochondrial",
  "gene": "UniProtKB:P13995",
  "term_id": "GO:0035999",
  "gene_symbol": "MTHFD2"
}